{
  "term_id": "GO:0005739",
  "gene_symbol": "COQ10B",
  "gene_name": "Coenzyme Q-binding protein COQ10 homolog B, mitochondrial",
  "gene": "UniProtKB:Q9H8M1",
  "term_label": "mitochondrion"
}